high-affinity IgM receptor activity [GO:0002172] (molecular function) Relationships: is a type of IgM receptor activity [GO:0001793] Definition: Combining with high affinity with an immunoglobulin of an IgM isotype via the Fc region, and transmitting the signal from one side of the membrane to the other to initiate a change in cell activity. Sources: GOC:hjd, GOC:signaling Also known as: high affinity IgM receptor activity